{
  "gene_name": "Prostate and testis expressed protein 4",
  "gene_symbol": "PATE4",
  "term_id": "UNKNOWN:0003",
  "gene": "UniProtKB:P0C8F1",
  "term_label": "Unknown cellular component"
}